{
  "gene_name": "Peptidoglycan recognition protein 3",
  "term_id": "GO:0006955",
  "gene_symbol": "PGLYRP3",
  "term_label": "immune response",
  "gene": "UniProtKB:Q96LB9"
}